purine ribonucleoside salvage [GO:0006166] (biological process) Definition: Any process which produces a purine nucleoside from derivatives of it, without de novo synthesis. Subtypes: GO:0006169, guanosine salvage [GO:0006179], inosine salvage [GO:0006190] Sources: GOC:jl Relationships: is a type of purine-containing compound salvage [GO:0043101]; is a type of GO:0043174; is a type of GO:0046129